{
  "gene_name": "Complement C1q-like protein 4",
  "term_id": "GO:0005615",
  "term_label": "extracellular space",
  "gene": "UniProtKB:Q86Z23",
  "gene_symbol": "C1QL4"
}